{
  "term_id": "GO:0004842",
  "gene": "UniProtKB:Q7L5Y9",
  "gene_name": "E3 ubiquitin-protein transferase MAEA",
  "term_label": "ubiquitin-protein transferase activity",
  "gene_symbol": "MAEA"
}